{
  "term_id": "UNKNOWN:0002",
  "gene_symbol": "TMEM175",
  "gene_name": "Endosomal_lysosomal proton channel TMEM175",
  "gene": "UniProtKB:Q9BSA9",
  "term_label": "Unknown biological process"
}